{
  "term_id": "UNKNOWN:0001",
  "gene_symbol": "HAPLN3",
  "term_label": "Unknown molecular function",
  "gene": "UniProtKB:Q96S86",
  "gene_name": "Hyaluronan and proteoglycan link protein 3"
}